viral process [GO:0016032] (biological process) Relationships: is a type of GO:0008150 Regulation: RO_0002213 by positive regulation of viral process [GO:0048524]; negatively regulated by negative regulation of viral process [GO:0048525]; regulated by GO:0050792 Definition: A multi-organism process in which a virus is a participant. The other participant is the host. Includes infection of a host cell, replication of the viral genome, and assembly of progeny virus particles. In some cases the viral genetic material may integrate into the host genome and only subsequently, under particular circumstances, 'complete' its life cycle. Sources: GOC:bf, GOC:jl, GOC:mah Note: See also the biological process terms 'viral infectious cycle ; GO:0019058' and 'lysogeny ; GO:0030069'. Subtypes: viral latency [GO:0019042], establishment of viral latency [GO:0019043], maintenance of viral latency [GO:0019044], latent virus replication [GO:0019045], release from viral latency [GO:0019046], GO:0019058, GO:0019061, virion assembly [GO:0019068], viral capsid assembly [GO:0019069], GO:0019070, viral genome packaging [GO:0019072], virus maturation [GO:0019075], viral release from host cell [GO:0019076], viral genome replication [GO:0019079], viral gene expression [GO:0019080], GO:0019081, viral protein processing [GO:0019082], viral transcription [GO:0019083], GO:0039639, GO:0039663, lysis of host organelle involved in viral entry into host cell [GO:0039664], permeabilization of host organelle membrane involved in viral entry into host cell [GO:0039665], GO:0039674, symbiont genome ejection through host cell envelope [GO:0039678], polyadenylation of viral mRNA by polymerase stuttering [GO:0039698], fusion of viral membrane with host outer nuclear membrane [GO:0039700], viral genome integration into host DNA [GO:0044826], viral capsid secondary envelopment [GO:0046745], viral budding [GO:0046755], viral mRNA export from host cell nucleus [GO:0046784], GO:0046786, transport of virus [GO:0046794], viral scaffold assembly and maintenance [GO:0046807], IRES-dependent viral translational initiation [GO:0075522], viral translational frameshifting [GO:0075523], ribosomal skipping [GO:0075524], viral translational termination-reinitiation [GO:0075525], cap snatching [GO:0075526], viral RNA editing [GO:0075527], GO:0098003, virus tail fiber assembly [GO:0098004], viral head-tail joining [GO:0098005], GO:0098045, superinfection exclusion [GO:0098669], virion maturation [GO:0098677], viral tropism switching [GO:0098678], GO:0098689, viral genome circularization [GO:0099009], GO:0099015, GO:0140755 Also known as: virus process, viral infection, virulence